{
  "gene_name": "Quinone oxidoreductase",
  "term_id": "GO:0003730",
  "term_label": "mRNA 3'-UTR binding",
  "gene_symbol": "CRYZ",
  "gene": "UniProtKB:Q08257"
}